Golgi calcium ion homeostasis [GO:0032468] (biological process) Definition: Any process involved in the maintenance of an internal steady state of calcium ions within the Golgi apparatus of a cell or between the Golgi and its surroundings. Also known as: Golgi calcium ion concentration regulation, calcium ion homeostasis in Golgi, regulation of Golgi calcium ion concentration, regulation of calcium ion concentration in Golgi Relationships: is a type of intracellular calcium ion homeostasis [GO:0006874]; occurs in GO:0005794 Sources: GOC:mah